{
  "gene_symbol": "MYCBP2",
  "term_id": "GO:0007411",
  "gene": "UniProtKB:O75592",
  "gene_name": "E3 ubiquitin-protein ligase MYCBP2",
  "term_label": "axon guidance"
}